{
  "gene_name": "Melanocyte-stimulating hormone receptor",
  "gene_symbol": "MC1R",
  "term_id": "GO:0005737",
  "gene": "UniProtKB:Q01726",
  "term_label": "cytoplasm"
}